endonucleolytic cleavage in 3'-ETS of tricistronic rRNA transcript (SSU-rRNA, 5.8S rRNA, LSU-rRNA) [GO:0000471] (biological process) Relationships: is a type of endonucleolytic cleavage of tricistronic rRNA transcript (SSU-rRNA, 5.8S rRNA, LSU-rRNA) [GO:0000479] References: PMID:10690410 Sources: GOC:krc Definition: Endonucleolytic cleavage within the 3'-External Transcribed Spacer (ETS) of a tricistronic rRNA transcript that contains the Small Subunit (SSU) rRNA, the 5.8S rRNA, and the Large Subunit (LSU) rRNA in that order from 5' to 3' along the primary transcript. In S. cerevisiae, endonucleolytic cleavage within the 3'-ETS of the pre-RNA, which may occur cotranscriptionally, is the first step in rRNA processing, and initiates a cascade of subsequent processing and modification events.